{
  "gene": "UniProtKB:Q9BRB3",
  "term_id": "UNKNOWN:0001",
  "term_label": "Unknown molecular function",
  "gene_symbol": "PIGQ",
  "gene_name": "Phosphatidylinositol N-acetylglucosaminyltransferase subunit Q"
}